{
  "term_id": "UNKNOWN:0002",
  "term_label": "Unknown biological process",
  "gene_symbol": "WDR5B",
  "gene": "UniProtKB:Q86VZ2",
  "gene_name": "WD repeat-containing protein 5B"
}